{
  "gene_name": "Histamine H4 receptor",
  "term_label": "adenylate cyclase-inhibiting G protein-coupled acetylcholine receptor signaling pathway",
  "gene_symbol": "HRH4",
  "term_id": "GO:0007197",
  "gene": "UniProtKB:Q9H3N8"
}